{
  "term_id": "GO:0003712",
  "gene_symbol": "MED1",
  "gene": "UniProtKB:Q15648",
  "gene_name": "Mediator of RNA polymerase II transcription subunit 1",
  "term_label": "transcription coregulator activity"
}